{
  "gene_symbol": "POMGNT2",
  "term_id": "GO:0097363",
  "term_label": "protein O-acetylglucosaminyltransferase activity",
  "gene_name": "Protein O-linked-mannose beta-1,4-N-acetylglucosaminyltransferase 2",
  "gene": "UniProtKB:Q8NAT1"
}